{
  "gene": "UniProtKB:Q8N912",
  "gene_name": "Nutritionally-regulated adipose and cardiac enriched protein homolog",
  "gene_symbol": "NRAC",
  "term_id": "UNKNOWN:0001",
  "term_label": "Unknown molecular function"
}